{
  "term_id": "GO:0042130",
  "gene": "UniProtKB:O75509",
  "gene_name": "Tumor necrosis factor receptor superfamily member 21",
  "term_label": "negative regulation of T cell proliferation",
  "gene_symbol": "TNFRSF21"
}